3'-UTR-mediated mRNA stabilization [GO:0070935] (biological process) Regulation: regulated by regulation of 3'-UTR-mediated mRNA stabilization [GO:1905868]; negatively regulated by negative regulation of 3'-UTR-mediated mRNA stabilization [GO:1905869]; positively regulated by positive regulation of 3'-UTR-mediated mRNA stabilization [GO:1905870] Relationships: is a type of GO:0048255 References: PMID:19029303 Sources: GOC:mah Definition: An mRNA stabilization process in which one or more RNA-binding proteins associate with the 3'-untranslated region (UTR) of an mRNA. Also known as: 3'-untranslated region-mediated mRNA stabilization